adenosine deaminase activity [GO:0004000] (MF) Definition: Catalysis of the reaction: adenosine + H2O = inosine + NH3. Also known as: adenosine deaminase reaction, adenosine aminohydrolase activity Relationships: is a type of hydrolase activity, acting on carbon-nitrogen (but not peptide) bonds, in cyclic amidines [GO:0016814]; is a type of deaminase activity [GO:0019239] Sources: RHEA:24408 Subtypes: tRNA-specific adenosine deaminase activity [GO:0008251]